{
  "gene": "UniProtKB:O95954",
  "gene_name": "Formimidoyltransferase-cyclodeaminase",
  "term_id": "GO:0030412",
  "term_label": "formimidoyltetrahydrofolate cyclodeaminase activity",
  "gene_symbol": "FTCD"
}